{
  "gene_name": "Myosin regulatory light chain 10",
  "gene_symbol": "MYL10",
  "term_id": "UNKNOWN:0002",
  "term_label": "Unknown biological process",
  "gene": "UniProtKB:Q9BUA6"
}